{
  "term_id": "GO:0050911",
  "gene_symbol": "OR12D3",
  "gene_name": "Olfactory receptor 12D3",
  "term_label": "detection of chemical stimulus involved in sensory perception of smell",
  "gene": "UniProtKB:Q9UGF7"
}